{
  "term_id": "GO:0005262",
  "gene_name": "Transient receptor potential cation channel subfamily V member 6",
  "gene_symbol": "TRPV6",
  "gene": "UniProtKB:Q9H1D0",
  "term_label": "calcium channel activity"
}